{
  "gene": "UniProtKB:Q5TCS8",
  "gene_name": "Adenylate kinase 9",
  "term_label": "CDP biosynthetic process",
  "term_id": "GO:0046705",
  "gene_symbol": "AK9"
}